{
  "gene_name": "G1_S-specific cyclin-E2",
  "gene": "UniProtKB:O96020",
  "gene_symbol": "CCNE2",
  "term_label": "cyclin E2-CDK2 complex",
  "term_id": "GO:0097135"
}